UDP-galactosyltransferase activity [GO:0035250] (molecular function) References: PMID:19858195 Definition: Catalysis of the transfer of a galactose group from UDP-galactose to an acceptor molecule. Subtypes: GO:0003831, GO:0003851, N-acetyllactosamine synthase activity [GO:0003945], fucosylgalactoside 3-alpha-galactosyltransferase activity [GO:0004381], lactose synthase activity [GO:0004461], UDP-galactose:glucosylceramide beta-1,4-galactosyltransferase activity [GO:0008489], GO:0008499, lipopolysaccharide 3-alpha-galactosyltransferase activity [GO:0008918], lipopolysaccharide-1,6-galactosyltransferase activity [GO:0008921], UDP-galactose:N-glycan beta-1,3-galactosyltransferase activity [GO:0010488], GO:0035496, digalactosyldiacylglycerol synthase activity [GO:0046481], GO:0046509, GO:0046525, inositol 3-alpha-galactosyltransferase activity [GO:0047216], galactosylxylosylprotein 3-beta-galactosyltransferase activity [GO:0047220], GO:0047221, GO:0047227, sucrose 6F-alpha-galactotransferase activity [GO:0047235], lactosylceramide beta-1,3-galactosyltransferase activity [GO:0047240], GO:0047255, sphingosine beta-galactosyltransferase activity [GO:0047258], glycosaminoglycan galactosyltransferase activity [GO:0047271], GO:0047276, sn-glycerol-3-phosphate 1-galactosyltransferase activity [GO:0047279], ganglioside galactosyltransferase activity [GO:0047915], procollagen galactosyltransferase activity [GO:0050211], lactosylceramide 4-alpha-galactosyltransferase activity [GO:0050512], tRNA-queuosine(34) galactosyltransferase activity [GO:0141125] Relationships: is a type of UDP-glycosyltransferase activity [GO:0008194]; is a type of galactosyltransferase activity [GO:0008378]